protein localization to cell-cell junction [GO:0150105] (biological process) Subtypes: protein localization to tricellular tight junction [GO:0061833], protein localization to adherens junction [GO:0071896], protein localization to basal ectoplasmic specialization [GO:0120145], GO:1902396 Relationships: is_a protein localization to cell junction [GO:1902414] Regulation: regulated by regulation of protein localization to cell-cell junction [GO:0150106]; RO_0002213 by GO:0150107; negatively regulated by negative regulation of protein localization to cell-cell junction [GO:0150119] Definition: A process in which a protein is transported to, or maintained, in a location within a cell-cell junction. References: PMID:26706435 Sources: GOC:aruk, GOC:bc